{
  "gene": "UniProtKB:O75027",
  "term_label": "transmembrane transport",
  "term_id": "GO:0055085",
  "gene_name": "Iron-sulfur clusters transporter ABCB7, mitochondrial",
  "gene_symbol": "ABCB7"
}